{
  "gene": "UniProtKB:P50053",
  "gene_name": "Ketohexokinase",
  "term_label": "regulation of glycogen metabolic process",
  "term_id": "GO:0070873",
  "gene_symbol": "KHK"
}